{
  "term_label": "P-type calcium transporter activity",
  "gene_name": "Sarcoplasmic_endoplasmic reticulum calcium ATPase 3",
  "gene": "UniProtKB:Q93084",
  "gene_symbol": "ATP2A3",
  "term_id": "GO:0005388"
}